{
  "gene_symbol": "CP",
  "term_label": "Unknown biological process",
  "gene": "UniProtKB:P00450",
  "gene_name": "Ceruloplasmin",
  "term_id": "UNKNOWN:0002"
}